{
  "gene": "UniProtKB:Q6ZP68",
  "term_id": "UNKNOWN:0002",
  "gene_name": "Putative protein ATP11AUN",
  "gene_symbol": "ATP11AUN",
  "term_label": "Unknown biological process"
}